{
  "gene_name": "Immunoglobulin heavy diversity 6-13 (Fragment)",
  "term_label": "Unknown biological process",
  "gene_symbol": "IGHD6-13",
  "gene": "UniProtKB:A0A1Y8EI39",
  "term_id": "UNKNOWN:0002"
}